{
  "gene_symbol": "RHOG",
  "gene_name": "Rho-related GTP-binding protein RhoG",
  "term_id": "GO:0005856",
  "gene": "UniProtKB:P84095",
  "term_label": "cytoskeleton"
}